{
  "gene_symbol": "CCR10",
  "term_label": "positive regulation of cytosolic calcium ion concentration",
  "gene_name": "C-C chemokine receptor type 10",
  "term_id": "GO:0007204",
  "gene": "UniProtKB:P46092"
}